{
  "gene_name": "Protein TANC1",
  "gene_symbol": "TANC1",
  "gene": "UniProtKB:Q9C0D5",
  "term_id": "GO:0099092",
  "term_label": "postsynaptic density, intracellular component"
}